{
  "term_id": "GO:0120020",
  "gene_symbol": "ABCG8",
  "gene_name": "ATP-binding cassette sub-family G member 8",
  "gene": "UniProtKB:Q9H221",
  "term_label": "cholesterol transfer activity"
}